{
  "gene_name": "ELAV-like protein 1",
  "gene_symbol": "ELAVL1",
  "gene": "UniProtKB:Q15717",
  "term_label": "Unknown cellular component",
  "term_id": "UNKNOWN:0003"
}